{
  "gene": "UniProtKB:Q96RS0",
  "term_label": "7-methylguanosine cap hypermethylation",
  "term_id": "GO:0036261",
  "gene_name": "Trimethylguanosine synthase",
  "gene_symbol": "TGS1"
}